{
  "term_id": "GO:0000028",
  "gene_name": "Ribosomal protein eS27-like",
  "gene_symbol": "RPS27L",
  "gene": "UniProtKB:Q71UM5",
  "term_label": "ribosomal small subunit assembly"
}